{
  "gene": "UniProtKB:Q9ULJ6",
  "term_id": "GO:0016925",
  "gene_name": "Zinc finger MIZ domain-containing protein 1",
  "term_label": "protein sumoylation",
  "gene_symbol": "ZMIZ1"
}